initial meiotic spindle pole body separation [GO:0140456] (biological process) References: PMID:31532702 Definition: The release of duplicated meiotic spindle pole bodies (SPBs). Relationships: is a type of spindle pole body separation [GO:0110100]; is a type of meiotic cell cycle process [GO:1903046] Also known as: initial spindle pole body separation involved in meiosis I, meiotic spindle pole body duplication